{
  "gene": "UniProtKB:Q14032",
  "term_id": "GO:0006637",
  "gene_name": "Bile acid-CoA:amino acid N-acyltransferase",
  "gene_symbol": "BAAT",
  "term_label": "acyl-CoA metabolic process"
}